{
  "term_label": "transmembrane transport",
  "gene_name": "Electrogenic sodium bicarbonate cotransporter 1",
  "gene": "UniProtKB:Q9Y6R1",
  "gene_symbol": "SLC4A4",
  "term_id": "GO:0055085"
}